division septum [GO:0000935] (cellular component) Also known as: septum surface, complete septum, cell septum surface Relationships: is a type of cell septum [GO:0030428]; is part of GO:0032153 Subtypes: primary cell septum [GO:0000936], GO:0051077 Definition: A cell septum which forms as part of the division site and functions in the compartmentalization of a cell into two daughter cells at division. A division septum spans a cell and does not allow exchange of organelles or cytoplasm between compartments. Sources: GOC:clt, GOC:vw